{
  "term_id": "GO:0043123",
  "gene": "UniProtKB:P50591",
  "term_label": "positive regulation of canonical NF-kappaB signal transduction",
  "gene_name": "Tumor necrosis factor ligand superfamily member 10",
  "gene_symbol": "TNFSF10"
}